{
  "gene_symbol": "TYRP1",
  "gene_name": "5,6-dihydroxyindole-2-carboxylic acid oxidase",
  "term_id": "GO:0030318",
  "gene": "UniProtKB:P17643",
  "term_label": "melanocyte differentiation"
}